{
  "term_label": "collagen metabolic process",
  "term_id": "GO:0032963",
  "gene_name": "Prolyl 3-hydroxylase 1",
  "gene_symbol": "P3H1",
  "gene": "UniProtKB:Q32P28"
}